{
  "gene": "UniProtKB:Q969G6",
  "term_label": "FMN biosynthetic process",
  "gene_name": "Riboflavin kinase",
  "gene_symbol": "RFK",
  "term_id": "GO:0009398"
}